NADH peroxidase activity [GO:0016692] (molecular function) Definition: Catalysis of the reaction: H2O2 + NADH + H+ = 2 H2O + NAD+. Relationships: is a type of peroxidase activity [GO:0004601] Sources: EC:1.11.1.1, RHEA:18509 Also known as: DPNH peroxidase activity, NAD peroxidase activity, NADH-peroxidase activity, NADH:hydrogen-peroxide oxidoreductase activity, diphosphopyridine nucleotide peroxidase activity, nicotinamide adenine dinucleotide peroxidase activity